{
  "gene_symbol": "NEXN-AS1",
  "term_label": "Unknown molecular function",
  "gene": "UniProtKB:Q8NBZ9",
  "gene_name": "Putative uncharacterized protein NEXN-AS1",
  "term_id": "UNKNOWN:0001"
}